positive regulation of adenylate cyclase-activating adrenergic receptor signaling pathway involved in heart process [GO:0140196] (biological process) Definition: Any process that activates or increases the frequency, rate or extent of an adenylate cyclase-activating adrenergic receptor signaling pathway involved in some heart process. Relationships: is_a positive regulation of multicellular organismal process [GO:0051240]; is_a positive regulation of adenylate cyclase-activating adrenergic receptor signaling pathway [GO:0071879]; is a type of positive regulation of adenylate cyclase-activating G protein-coupled receptor signaling pathway [GO:0106071]; positively regulates GO:0086023 Sources: GOC:BHF, GOC:BHF_miRNA, GOC:rph